{
  "gene_symbol": "FN3K",
  "term_id": "GO:0030389",
  "term_label": "fructosamine metabolic process",
  "gene_name": "Fructosamine-3-kinase",
  "gene": "UniProtKB:Q9H479"
}